{
  "term_label": "Unknown molecular function",
  "gene": "UniProtKB:A0A087WSY6",
  "term_id": "UNKNOWN:0001",
  "gene_symbol": "IGKV3D-15",
  "gene_name": "Immunoglobulin kappa variable 3D-15"
}